{
  "gene_symbol": "SHROOM1",
  "gene_name": "Protein Shroom1",
  "gene": "UniProtKB:Q2M3G4",
  "term_id": "GO:0005912",
  "term_label": "adherens junction"
}